ditrans,polycis-polyprenyl diphosphate synthase [(2E,6E)-farnesyl diphosphate specific] activity [GO:0045547] (molecular function) Relationships: is a type of prenyl diphosphate synthase activity [GO:0120531] Also known as: dehydrodolichyl diphosphate synthase activity Definition: Catalysis of the reaction: (2E,6E)-farnesyl diphosphate + n isopentenyl diphosphate = a di-trans,poly-cis-polyprenyl diphosphate + n diphosphate. Subtypes: ditrans,polycis-undecaprenyl-diphosphate synthase [(2E,6E)-farnesyl-diphosphate specific] activity [GO:0008834] References: PMID:9858571 Sources: RHEA:53008